nuclear inner membrane organization [GO:0071765] (biological process) Definition: A process that is carried out at the cellular level which results in the assembly, arrangement of constituent parts, or disassembly of the nuclear inner membrane. Also known as: nuclear inner membrane organisation, nuclear inner membrane organization and biogenesis Sources: GOC:mah Relationships: is a type of nuclear membrane organization [GO:0071763]